{
  "term_id": "GO:0005814",
  "gene_symbol": "SAXO2",
  "gene_name": "Stabilizer of axonemal microtubules 2",
  "gene": "UniProtKB:Q658L1",
  "term_label": "centriole"
}